symbiont genome ejection through host cell envelope, short tail mechanism [GO:0099002] (biological process) Also known as: viral short tail ejection system, viral genome ejection through host cell envelope, short tail mechanism Relationships: is a type of symbiont genome ejection through host cell envelope [GO:0039678] Definition: Entry of a symbiont's genome into the host cell through the host cell envelope via a short tail ejection system consisting a central tube, the connector which attaches the tail to the phage capsid and releases inner core proteins. Upon binding to the host cell surface, the phage displays a tube-like extension of its short tail that penetrates both host membranes. This tail extension comes from the release of viral core proteins with channel forming properties. Occurs in non-enveloped prokaryotic viruses. References: PMID:22297513 Sources: GOC:dos, VZ:3954